{
  "term_id": "GO:0005886",
  "gene_name": "Protein PALS1",
  "gene_symbol": "PALS1",
  "term_label": "plasma membrane",
  "gene": "UniProtKB:Q8N3R9"
}